{
  "term_label": "regulation of epidermal cell division",
  "term_id": "GO:0010482",
  "gene": "UniProtKB:Q8NAX2",
  "gene_symbol": "KDF1",
  "gene_name": "Keratinocyte differentiation factor 1"
}